{
  "term_label": "receptor complex",
  "gene": "UniProtKB:P22607",
  "gene_name": "Fibroblast growth factor receptor 3",
  "gene_symbol": "FGFR3",
  "term_id": "GO:0043235"
}